{
  "gene_name": "Protein LBH",
  "term_id": "GO:0005634",
  "gene_symbol": "LBH",
  "term_label": "nucleus",
  "gene": "UniProtKB:Q53QV2"
}